{
  "gene_symbol": "C17orf67",
  "gene": "UniProtKB:Q0P5P2",
  "gene_name": "Uncharacterized protein C17orf67",
  "term_label": "Unknown molecular function",
  "term_id": "UNKNOWN:0001"
}